{
  "gene_symbol": "PDGFRB",
  "term_label": "positive regulation of smooth muscle cell migration",
  "gene_name": "Platelet-derived growth factor receptor beta",
  "term_id": "GO:0014911",
  "gene": "UniProtKB:P09619"
}